{
  "gene": "UniProtKB:P26599",
  "gene_symbol": "PTBP1",
  "term_id": "GO:0045595",
  "term_label": "regulation of cell differentiation",
  "gene_name": "Polypyrimidine tract-binding protein 1"
}